{
  "term_id": "GO:0071949",
  "term_label": "FAD binding",
  "gene_name": "Cyanocobalamin reductase _ alkylcobalamin dealkylase",
  "gene": "UniProtKB:Q9Y4U1",
  "gene_symbol": "MMACHC"
}